sulfopyruvate decarboxylase activity [GO:0050545] (molecular function) Definition: Catalysis of the reaction: 3-sulfopyruvate + H+ = CO2 + sulfoacetaldehyde. Sources: EC:4.1.1.79, RHEA:20948 Relationships: is a type of carboxy-lyase activity [GO:0016831] Also known as: sulphopyruvate decarboxylase activity, sulfopyruvate carboxy-lyase (2-sulfoacetaldehyde-forming), sulfopyruvate carboxy-lyase activity